{
  "gene_symbol": "ADGRG6",
  "term_id": "GO:0005886",
  "gene_name": "Adhesion G-protein coupled receptor G6",
  "term_label": "plasma membrane",
  "gene": "UniProtKB:Q86SQ4"
}